{
  "gene_symbol": "SEL1L2",
  "gene_name": "Protein sel-1 homolog 2",
  "term_label": "Unknown molecular function",
  "gene": "UniProtKB:Q5TEA6",
  "term_id": "UNKNOWN:0001"
}